{
  "gene": "UniProtKB:Q9BQG0",
  "term_id": "UNKNOWN:0002",
  "gene_symbol": "MYBBP1A",
  "term_label": "Unknown biological process",
  "gene_name": "Myb-binding protein 1A"
}